{
  "term_id": "GO:0005886",
  "gene_symbol": "BEST3",
  "gene": "UniProtKB:Q8N1M1",
  "gene_name": "Bestrophin-3",
  "term_label": "plasma membrane"
}